mitotic spindle pole body duplication [GO:1903087] (BP) Sources: GOC:TermGenie, GOC:mtg_cell_cycle, GO_REF:0000060 Also known as: spindle pole body assembly involved in mitotic cell cycle, spindle pole body biogenesis involved in mitotic cell cycle, spindle pole body biosynthesis involved in mitotic cell cycle, spindle pole body duplication associated with nuclear envelope involved in mitotic cell cycle, spindle pole body duplication in cytoplasm involved in mitotic cell cycle, spindle pole body duplication involved in mitotic cell cycle, spindle pole body formation involved in mitotic cell cycle, spindle pole body replication involved in mitotic cell cycle Definition: Any spindle pole body duplication that is involved in the mitotic cell cycle. Relationships: is a type of spindle pole body duplication [GO:0030474]; is a type of mitotic cell cycle process [GO:1903047]